{
  "gene_name": "Uncharacterized protein DKFZp781C0719",
  "gene": "UniProtKB:Q68DW6",
  "term_label": "Unknown cellular component",
  "gene_symbol": "DKFZp781C0719",
  "term_id": "UNKNOWN:0003"
}